{
  "gene_name": "Tumor necrosis factor ligand superfamily member 15",
  "term_id": "GO:0005615",
  "gene": "UniProtKB:O95150",
  "gene_symbol": "TNFSF15",
  "term_label": "extracellular space"
}